lipoprotein particle binding [GO:0071813] (molecular function) Relationships: is_a protein-lipid complex binding [GO:0071814] Sources: GOC:BHF, GOC:mah Subtypes: high-density lipoprotein particle binding [GO:0008035], low-density lipoprotein particle binding [GO:0030169], very-low-density lipoprotein particle binding [GO:0034189], chylomicron binding [GO:0035478], intermediate-density lipoprotein particle binding [GO:0071815] Also known as: plasma lipoprotein particle binding, lipoprotein binding, plasma lipoprotein binding Definition: Binding to a lipoprotein particle. A lipoprotein particle, also known as a lipoprotein, is a clathrate complex consisting of a lipid enwrapped in a protein host without covalent binding in such a way that the complex has a hydrophilic outer surface consisting of all the protein and the polar ends of any phospholipids.